{
  "gene_name": "Methenyltetrahydrofolate synthase domain-containing protein",
  "gene": "UniProtKB:Q2M296",
  "term_id": "GO:0005737",
  "gene_symbol": "MTHFSD",
  "term_label": "cytoplasm"
}